{
  "term_id": "GO:0019216",
  "gene_name": "Angiopoietin-like protein 8",
  "term_label": "regulation of lipid metabolic process",
  "gene_symbol": "ANGPTL8",
  "gene": "UniProtKB:Q6UXH0"
}